{
  "gene": "UniProtKB:P15153",
  "term_label": "GTPase activity",
  "gene_symbol": "RAC2",
  "gene_name": "Ras-related C3 botulinum toxin substrate 2",
  "term_id": "GO:0003924"
}